dormancy entry of symbiont in host [GO:0085014] (biological process) Definition: Entry into a dormant state of the symbiont within the host organism. Relationships: is a type of dormancy process [GO:0022611]; is a type of development of symbiont in host [GO:0044114] Sources: GOC:jl